{
  "gene_symbol": "CEP170P1",
  "gene_name": "Cep170-like protein",
  "gene": "UniProtKB:Q96L14",
  "term_label": "Unknown cellular component",
  "term_id": "UNKNOWN:0003"
}